{
  "term_id": "UNKNOWN:0001",
  "term_label": "Unknown molecular function",
  "gene_name": "Transferrin receptor protein 1",
  "gene": "UniProtKB:P02786",
  "gene_symbol": "TFRC"
}